Ser-tRNA(Ala) deacylase activity [GO:0002196] (MF) References: PMID:21285375 Sources: GOC:hjd Definition: Catalysis of the hydrolysis of misacylated Ser-tRNA(Ala). Relationships: is a type of aminoacyl-tRNA deacylase activity [GO:0002161]